intron homing [GO:0006314] (biological process) Definition: Lateral transfer of an intron to a homologous allele that lacks the intron, mediated by a site-specific endonuclease encoded within the mobile intron. Subtypes: homing of group II introns [GO:0006315], GO:0006316 References: PMID:10487208 Relationships: is a type of DNA recombination [GO:0006310]